phytochelatin 4 import into vacuole [GO:0036248] (biological process) Also known as: PC4 import into vacuole Definition: The directed movement of phytochelatin 4 (PC4) into the vacuole. Phytochelatin 4 is a glutathione-related peptide composed of (gamma-Glu-Cys)n-Gly where n=4, and where the Glu and Cys residues are linked through a gamma-carboxylamide bond. References: PMID:19001374 Sources: GOC:al Relationships: is a type of oligopeptide transmembrane transport [GO:0035672]; is a type of phytochelatin import into vacuole [GO:0071995]